{
  "term_label": "Unknown molecular function",
  "term_id": "UNKNOWN:0001",
  "gene": "UniProtKB:A0N4X2",
  "gene_name": "Possible J 40 gene segment (Fragment)",
  "gene_symbol": "TRAJ40"
}